{
  "term_label": "thiamine pyrophosphate binding",
  "gene_symbol": "TKT",
  "gene": "UniProtKB:P29401",
  "term_id": "GO:0030976",
  "gene_name": "Transketolase"
}